{
  "term_label": "Unknown biological process",
  "gene_symbol": "MARVELD3",
  "gene_name": "MARVEL domain-containing protein 3",
  "gene": "UniProtKB:Q96A59",
  "term_id": "UNKNOWN:0002"
}